maltose:proton symporter activity [GO:0005364] (molecular function) Definition: Enables the transfer of a solute or solutes from one side of a membrane to the other according to the reaction: maltose(out) + H+(out) = maltose(in) + H+(in). Relationships: is_a carbohydrate:proton symporter activity [GO:0005351]; is a type of maltose transmembrane transporter activity [GO:0005363] Sources: TC:2.A.1.1.10 Also known as: hydrogen/maltose transporter activity, maltose permease, maltose:hydrogen symporter activity